{
  "term_id": "GO:0000123",
  "term_label": "histone acetyltransferase complex",
  "gene_symbol": "JADE2",
  "gene": "UniProtKB:Q9NQC1",
  "gene_name": "E3 ubiquitin-protein ligase Jade-2"
}